polyamine acetylation [GO:0032917] (biological process) Relationships: is a type of polyamine metabolic process [GO:0006595] Sources: GOC:mlg Subtypes: spermidine acetylation [GO:0032918], GO:0032919, putrescine acetylation [GO:0032920] Definition: The modification of polyamines by addition of acetyl groups.